C-fiber [GO:0044299] (cellular component) Definition: The axon of a dorsal root ganglion cell that are responsive to pain and temperature. C-fibers are small in diameter (0.2-1.5 um) and unmyelinated. Sources: NIF_Subcellular:nlx_subcell_20090210 Also known as: C-fibre Relationships: is a type of axon [GO:0030424]